plastid inner membrane [GO:0009528] (CC) Definition: The inner, i.e. lumen-facing, lipid bilayer of the plastid envelope; also faces the plastid stroma. Sources: GOC:lr Relationships: is a type of GO:0019866; is a type of plastid membrane [GO:0042170] Subtypes: chloroplast inner membrane [GO:0009706], chromoplast inner membrane [GO:0031899], amyloplast inner membrane [GO:0033098], cyanelle inner membrane [GO:0036012]